L-histidine, sodium:proton antiporter activity [GO:0140832] (molecular function) Relationships: is a type of L-histidine transmembrane transporter activity [GO:0005290]; is a type of sodium:proton antiporter activity [GO:0015385]; is a type of azole:proton antiporter activity [GO:0045119]; is a type of amino acid:monoatomic cation antiporter activity [GO:0140848] References: PMID:10619430, PMID:11742981 Definition: Enables the transfer of a solute or solutes from one side of a membrane to the other according to the reaction: H+(in) + L-histidine(out) + Na+(out) = H+(out) + L-histidine(in) + Na+(in).